{
  "gene_symbol": "SPTBN1",
  "term_label": "plasma membrane",
  "gene": "UniProtKB:Q01082",
  "gene_name": "Spectrin beta chain, non-erythrocytic 1",
  "term_id": "GO:0005886"
}